{
  "term_id": "GO:0004521",
  "gene_name": "Integrator complex subunit 11",
  "term_label": "RNA endonuclease activity",
  "gene_symbol": "INTS11",
  "gene": "UniProtKB:Q5TA45"
}